non-photoreactive DNA repair [GO:0010213] (biological process) Definition: A DNA repair process that is involved in repairing UV-induced DNA damage under non-photoreactivating conditions. The mechanism by which this repair process operates has not yet been completely elucidated. Sources: GOC:syr Relationships: is a type of DNA repair [GO:0006281] Also known as: light-independent DNA repair